{
  "term_label": "recycling endosome",
  "gene": "UniProtKB:Q8NB49",
  "gene_symbol": "ATP11C",
  "gene_name": "Phospholipid-transporting ATPase IG",
  "term_id": "GO:0055037"
}